{
  "term_label": "cleavage furrow",
  "term_id": "GO:0032154",
  "gene_name": "Myosin light chain kinase, smooth muscle",
  "gene": "UniProtKB:Q15746",
  "gene_symbol": "MYLK"
}